cellular response to type III interferon [GO:0071358] (biological process) Definition: Any process that results in a change in state or activity of a cell (in terms of movement, secretion, enzyme production, gene expression, etc.) as a result of a type III interferon stimulus. Interferon lambda is the only member of the type III interferon found so far. Sources: GOC:mah Also known as: cellular response to type III IFN, cellular response to interferon-lambda Relationships: is a type of response to type III interferon [GO:0034342]; is a type of cellular response to cytokine stimulus [GO:0071345]